{
  "gene_name": "Putative uncharacterized protein encoded by MAPKAPK5-AS1",
  "gene_symbol": "MAPKAPK5-AS1",
  "term_label": "Unknown molecular function",
  "gene": "UniProtKB:Q8N8E1",
  "term_id": "UNKNOWN:0001"
}